{
  "term_id": "UNKNOWN:0001",
  "term_label": "Unknown molecular function",
  "gene_name": "UDP-GlcNAc:betaGal beta-1,3-N-acetylglucosaminyltransferase-like protein 1",
  "gene": "UniProtKB:Q67FW5",
  "gene_symbol": "B3GNTL1"
}